{
  "term_id": "GO:0016020",
  "gene_symbol": "PCSK6",
  "term_label": "membrane",
  "gene_name": "Proprotein convertase subtilisin_kexin type 6",
  "gene": "UniProtKB:P29122"
}